{
  "term_id": "GO:0008250",
  "gene_symbol": "DAD1",
  "term_label": "oligosaccharyltransferase complex",
  "gene_name": "Dolichyl-diphosphooligosaccharide--protein glycosyltransferase subunit DAD1",
  "gene": "UniProtKB:P61803"
}